{
  "gene_symbol": "DNAJB1",
  "gene_name": "DnaJ homolog subfamily B member 1",
  "gene": "UniProtKB:P25685",
  "term_id": "GO:0005829",
  "term_label": "cytosol"
}